{
  "gene_symbol": "GJD2",
  "gene": "UniProtKB:Q9UKL4",
  "gene_name": "Gap junction delta-2 protein",
  "term_id": "GO:0005243",
  "term_label": "gap junction channel activity"
}